{
  "gene_symbol": "AGRN",
  "gene": "UniProtKB:O00468",
  "term_id": "GO:0030297",
  "term_label": "transmembrane receptor protein tyrosine kinase activator activity",
  "gene_name": "Agrin"
}